{
  "gene": "UniProtKB:Q96PY0",
  "gene_name": "Putative uncharacterized protein PSMG3-AS1",
  "term_id": "UNKNOWN:0001",
  "term_label": "Unknown molecular function",
  "gene_symbol": "PSMG3-AS1"
}